{
  "term_label": "endosome to lysosome transport",
  "term_id": "GO:0008333",
  "gene_symbol": "VPS18",
  "gene": "UniProtKB:Q9P253",
  "gene_name": "Vacuolar protein sorting-associated protein 18 homolog"
}